{
  "term_label": "serotonin:sodium:chloride symporter activity",
  "gene_name": "Synaptic vesicular amine transporter",
  "term_id": "GO:0005335",
  "gene_symbol": "SLC18A2",
  "gene": "UniProtKB:Q05940"
}